cytoplasmic periphery of the nuclear pore complex [GO:1990723] (CC) Definition: Cytoplasm situated in close proximity to a nuclear pore complex. Also known as: associated with the nuclear pore Relationships: is a type of perinuclear region of cytoplasm [GO:0048471] References: PMID:9398662